{
  "gene_symbol": "SMIM7",
  "term_id": "UNKNOWN:0001",
  "term_label": "Unknown molecular function",
  "gene_name": "Small integral membrane protein 7",
  "gene": "UniProtKB:Q9BQ49"
}